{
  "term_id": "UNKNOWN:0002",
  "gene": "UniProtKB:Q8TCG1",
  "gene_name": "Protein CIP2A",
  "term_label": "Unknown biological process",
  "gene_symbol": "CIP2A"
}